{
  "term_id": "GO:0005737",
  "gene_name": "Inosine-5'-monophosphate dehydrogenase 1",
  "gene_symbol": "IMPDH1",
  "term_label": "cytoplasm",
  "gene": "UniProtKB:P20839"
}